symbiont genome entry into host cell via pore formation in plasma membrane [GO:0044694] (biological process) Definition: Entry of a symbiont's genome into a host cell by a pore formed by the symbiont in the host cell. Examples of this process include injection by a non-enveloped virus of the viral genome into the host cytoplasm, usually mediated by a viral pore-forming peptide associated with the viral capsid or bacteriophage tail. Sources: GOC:jl, VZ:979 Also known as: viral genome translocation, pore-mediated entry of viral genome into host cell, viral genome delivery via icosahedral vertex, viral pore-forming protein, membrane puncture-mediated penetration of viral genome into host cell, pore-mediated penetration of viral genome into host cell, viral entry via genome injection Note: This mechanism is used by animal viruses such as poliovirus. Various tailed bacteriophages also carry specialized proteins which open a pore or a channel in the host membrane(s) to allow genome delivery into host cytoplasm. Relationships: is a type of symbiont-mediated perturbation of host membrane [GO:0141171]; is part of symbiont entry into host cell [GO:0046718]